{
  "term_id": "GO:0000981",
  "gene_symbol": "ETV2",
  "gene_name": "ETS translocation variant 2",
  "term_label": "DNA-binding transcription factor activity, RNA polymerase II-specific",
  "gene": "UniProtKB:O00321"
}